{
  "gene": "UniProtKB:Q6EMB2",
  "term_id": "GO:0070740",
  "gene_name": "Tubulin polyglutamylase TTLL5",
  "gene_symbol": "TTLL5",
  "term_label": "tubulin-glutamic acid ligase activity"
}